{
  "term_label": "Unknown biological process",
  "gene_name": "KATNB1-like protein 1",
  "gene_symbol": "KATNBL1",
  "gene": "UniProtKB:Q9H079",
  "term_id": "UNKNOWN:0002"
}